{
  "term_id": "GO:0032926",
  "gene": "UniProtKB:P19883",
  "term_label": "negative regulation of activin receptor signaling pathway",
  "gene_symbol": "FST",
  "gene_name": "Follistatin"
}